{
  "gene": "UniProtKB:Q6ZRT6",
  "gene_name": "Proline-rich protein 23B",
  "term_id": "UNKNOWN:0002",
  "term_label": "Unknown biological process",
  "gene_symbol": "PRR23B"
}